proteasome regulatory particle, base subcomplex [GO:0008540] (cellular component) Subtypes: nuclear proteasome regulatory particle, base subcomplex [GO:0031610], cytosolic proteasome regulatory particle, base subcomplex [GO:0031612] Sources: GOC:mtg_sensu, GOC:rb Definition: The subcomplex of the proteasome regulatory particle that directly associates with the proteasome core complex. Relationships: is a type of protein-containing complex [GO:0032991]; is part of GO:0005838